{
  "gene_name": "Metal cation symporter ZIP8",
  "term_id": "GO:0140410",
  "term_label": "monoatomic cation:bicarbonate symporter activity",
  "gene_symbol": "SLC39A8",
  "gene": "UniProtKB:Q9C0K1"
}